{
  "gene_symbol": "DDX59",
  "gene_name": "Probable ATP-dependent RNA helicase DDX59",
  "gene": "UniProtKB:Q5T1V6",
  "term_id": "GO:0003724",
  "term_label": "RNA helicase activity"
}